{
  "gene_symbol": "KIAA0319L",
  "gene": "UniProtKB:Q8IZA0",
  "term_label": "cytoplasmic vesicle",
  "term_id": "GO:0031410",
  "gene_name": "Dyslexia-associated protein KIAA0319-like protein"
}